{
  "gene_name": "TP53-regulated inhibitor of apoptosis 1",
  "term_id": "GO:0097035",
  "gene_symbol": "TRIAP1",
  "term_label": "regulation of membrane lipid distribution",
  "gene": "UniProtKB:O43715"
}